nectary development [GO:0010254] (biological process) Sources: GOC:lr Definition: The process whose specific outcome is the progression of the floral nectaries over time, from its formation to the mature structure. Relationships: is a type of GO:0003006; is a type of anatomical structure development [GO:0048856]; is part of GO:0009908